{
  "gene_symbol": "TGM3",
  "term_id": "GO:0003810",
  "gene_name": "Protein-glutamine gamma-glutamyltransferase E",
  "term_label": "protein-glutamine gamma-glutamyltransferase activity",
  "gene": "UniProtKB:Q08188"
}